MECO complex [GO:0002929] (cellular component) References: PMID:20508642 Sources: GOC:hjd Also known as: meta-coactivator complex Relationships: is a type of protein-containing complex [GO:0032991]; BFO_0000051 mediator complex [GO:0016592]; has part ATAC complex [GO:0140672] Definition: A highly stable complex composed of the ATAC complex and the mediator complex (also called TRAP or MED). MECO binds and regulates the transcription of a subset of non-coding RNAs transcribed by RNA polymerase II.